{
  "gene_symbol": "BARGIN",
  "gene_name": "Bargin",
  "term_label": "regulation of actin cytoskeleton organization",
  "term_id": "GO:0032956",
  "gene": "UniProtKB:Q6ZT62"
}